primary active transmembrane transporter activity [GO:0015399] (molecular function) Definition: Enables the transfer of a solute from one side of a membrane to the other, up the solute's concentration gradient, by binding the solute and undergoing a series of conformational changes. Transport works equally well in either direction and is powered by a primary energy source. Primary energy sources known to be coupled to transport are chemical such as ATP hydrolysis, redox energy and photon energy. References: PMID:31613498 Sources: GOC:mtg_transport Also known as: primary active transporter Relationships: is a type of active transmembrane transporter activity [GO:0022804]; has part catalytic activity [GO:0003824] Subtypes: GO:0015451, methyl transfer-driven active transmembrane transporter activity [GO:0015452], GO:0015453, GO:0022853, GO:0042626